DNA replication-dependent chromatin assembly [GO:0006335] (biological process) References: PMID:28053344 Sources: GOC:mah Relationships: is a type of chromatin organization [GO:0006325] Also known as: DNA replication-dependent nucleosome assembly, DNA replication-dependent chromatin organization, DNA replication-dependent nucleosome organisation, DNA replication-dependent nucleosome organization Definition: The formation of nucleosomes on newly synthesized DNA, coupled to strand elongation.